monoatomic cation transmembrane transport [GO:0098655] (biological process) Definition: The process in which a monoatomic cation is transported across a membrane. Monatomic cations (also called simple cations) are positively charged ions consisting of exactly one atom. Sources: GOC:dos, GOC:vw Also known as: cation transmembrane transport, ATP hydrolysis coupled cation transmembrane transport Relationships: is a type of GO:0006812; is a type of monoatomic ion transmembrane transport [GO:0034220] Subtypes: cobalt ion transport [GO:0006824], mercury ion transport [GO:0015694], iron ion transmembrane transport [GO:0034755], copper ion transmembrane transport [GO:0035434], nickel cation transmembrane transport [GO:0035444], sodium ion transmembrane transport [GO:0035725], cadmium ion transmembrane transport [GO:0070574], calcium ion transmembrane transport [GO:0070588], manganese ion transmembrane transport [GO:0071421], GO:0071577, potassium ion transmembrane transport [GO:0071805], GO:0090452, proton transmembrane transport [GO:1902600], GO:1902601, GO:1903830 Regulation: regulated by GO:1904062; negatively regulated by negative regulation of cation transmembrane transport [GO:1904063]; positively regulated by positive regulation of cation transmembrane transport [GO:1904064]